response to macrophage colony-stimulating factor [GO:0036005] (biological process) Relationships: is a type of response to cytokine [GO:0034097] References: PMID:14687666 Sources: GOC:yaf Subtypes: cellular response to macrophage colony-stimulating factor stimulus [GO:0036006] Also known as: response to M-CSF, response to macrophage colony-stimulating factor stimulus Definition: Any process that results in a change in state or activity of a cell or an organism (in terms of movement, secretion, enzyme production, gene expression, etc.) as a result of a macrophage colony-stimulating factor stimulus. Regulation: regulated by GO:1903969; negatively regulated by negative regulation of response to macrophage colony-stimulating factor [GO:1903970]; positively regulated by GO:1903971